{
  "term_id": "GO:0004827",
  "gene": "UniProtKB:P07814",
  "gene_symbol": "EPRS1",
  "gene_name": "Bifunctional glutamate_proline--tRNA ligase",
  "term_label": "proline-tRNA ligase activity"
}